{
  "gene": "UniProtKB:Q6PJP8",
  "gene_symbol": "DCLRE1A",
  "term_id": "GO:0035312",
  "term_label": "5'-3' DNA exonuclease activity",
  "gene_name": "DNA cross-link repair 1A protein"
}